{
  "gene": "UniProtKB:Q16537",
  "term_id": "GO:0005829",
  "gene_name": "Serine_threonine-protein phosphatase 2A 56 kDa regulatory subunit epsilon isoform",
  "gene_symbol": "PPP2R5E",
  "term_label": "cytosol"
}